{
  "gene_name": "1-phosphatidylinositol 4,5-bisphosphate phosphodiesterase beta-4",
  "gene_symbol": "PLCB4",
  "term_id": "GO:0051209",
  "gene": "UniProtKB:Q15147",
  "term_label": "release of sequestered calcium ion into cytosol"
}